{
  "term_id": "GO:0005794",
  "gene_symbol": "MMGT1",
  "term_label": "Golgi apparatus",
  "gene_name": "ER membrane protein complex subunit 5",
  "gene": "UniProtKB:Q8N4V1"
}